{
  "gene": "UniProtKB:Q9UHL9",
  "gene_name": "General transcription factor II-I repeat domain-containing protein 1",
  "term_label": "Unknown biological process",
  "gene_symbol": "GTF2IRD1",
  "term_id": "UNKNOWN:0002"
}